{
  "term_label": "inward rectifier potassium channel activity",
  "gene": "UniProtKB:Q9H252",
  "term_id": "GO:0005242",
  "gene_name": "Potassium voltage-gated channel subfamily H member 6",
  "gene_symbol": "KCNH6"
}